{
  "gene_name": "Serine_threonine-protein kinase LATS2",
  "gene_symbol": "LATS2",
  "term_id": "GO:0005634",
  "term_label": "nucleus",
  "gene": "UniProtKB:Q9NRM7"
}